{
  "gene_symbol": "NOP56",
  "gene": "UniProtKB:O00567",
  "gene_name": "Nucleolar protein 56",
  "term_label": "snoRNA binding",
  "term_id": "GO:0030515"
}